posterior lateral line neuromast cupula development [GO:0048921] (biological process) Sources: ISBN:0125296509 Definition: The process whose specific outcome is the progression of the posterior lateral line neuromast cupula over time, from its formation to the mature structure. The cupula is secreted by mantle cells and the ciliary bundles of all of the hair cells of the neuromast are embedded in it. The cupula provides a mechanical linkage between the hair cells and the external hydrodynamic environment. The cupula of superficial neuromasts grows continuously, while the height of the cupula of canal neuromasts is limited by canal diameter. Relationships: is_a cupula development [GO:0048887]; is part of posterior lateral line neuromast development [GO:0048919]